{
  "gene_symbol": "GABRA5",
  "term_label": "GABA-gated chloride ion channel activity",
  "gene": "UniProtKB:P31644",
  "term_id": "GO:0022851",
  "gene_name": "Gamma-aminobutyric acid receptor subunit alpha-5"
}